{
  "gene_name": "Cytoplasmic polyadenylation element-binding protein 4",
  "gene_symbol": "CPEB4",
  "term_id": "GO:0005634",
  "gene": "UniProtKB:Q17RY0",
  "term_label": "nucleus"
}